2-(3-amino-3-carboxypropyl)histidine synthase complex [GO:0120513] (cellular component) Definition: A protein complex capable of catalysing the transfer of the 3-amino-3-carboxypropyl group from S-adenosyl-L-methionine (SAM) to the histidine residue of translation elongation factor 2 (EF2), which is the first step in the biosynthesis of diphthamide. The complex is a Dph2 homodimer in archaea and a Dph1-Dph2 heterodimer in eukaryotes. References: PMID:24422557, PMID:31463593 Sources: GOC:sjm Also known as: Dph1-Dph2 complex Relationships: is a type of transferase complex [GO:1990234]